UCA codon-amino acid adaptor activity [GO:0033407] (molecular function) Note: Note that in the standard genetic code, TCA codes for serine. Relationships: is a type of triplet codon-amino acid adaptor activity [GO:0030533] Also known as: TCA codon-amino acid adaptor activity, serine tRNA Sources: GOC:mah Definition: A triplet codon-amino acid adaptor activity that recognizes a UCA codon.